phosphoribulokinase activity [GO:0008974] (molecular function) Sources: EC:2.7.1.19, RHEA:19365 Relationships: is a type of kinase activity [GO:0016301]; is a type of GO:0016773 Also known as: 5-phosphoribulose kinase activity, ATP:D-ribulose-5-phosphate 1-phosphotransferase activity, PKK, PRK, PRuK, phosphopentokinase activity, phosphoribulokinase (phosphorylating), ribulose phosphate kinase activity, ribulose-5-phosphate kinase activity Definition: Catalysis of the reaction: D-ribulose 5-phosphate + ATP = D-ribulose 1,5-bisphosphate + ADP + 2 H+.